{
  "term_id": "UNKNOWN:0001",
  "term_label": "Unknown molecular function",
  "gene_name": "Vacuolar protein sorting-associated protein 35",
  "gene_symbol": "VPS35",
  "gene": "UniProtKB:Q96QK1"
}